{
  "gene_symbol": "SEPSECS",
  "gene": "UniProtKB:Q9HD40",
  "term_label": "tRNA binding",
  "term_id": "GO:0000049",
  "gene_name": "O-phosphoseryl-tRNA(Sec) selenium transferase"
}